{
  "term_label": "Unknown cellular component",
  "term_id": "UNKNOWN:0003",
  "gene_name": "2-(3-amino-3-carboxypropyl)histidine synthase subunit 2",
  "gene": "UniProtKB:Q9BQC3",
  "gene_symbol": "DPH2"
}